multivesicular body membrane disassembly [GO:0034496] (biological process) Relationships: is a type of membrane disassembly [GO:0030397]; BFO_0000050 GO:0036257 Also known as: MVB membrane disassembly Definition: The controlled breakdown of the membranes of multivesicular bodies. Sources: GOC:rb